{
  "gene_symbol": "TOPBP1",
  "term_id": "GO:0140463",
  "gene_name": "DNA topoisomerase 2-binding protein 1",
  "term_label": "chromatin-protein adaptor activity",
  "gene": "UniProtKB:Q92547"
}